positive regulation of anoikis [GO:2000210] (biological process) Definition: Any process that activates or increases the frequency, rate or extent of anoikis. Sources: GOC:mah Also known as: positive regulation of detachment induced cell death, positive regulation of suspension induced apoptosis Relationships: is a type of GO:0043065; is a type of GO:2000209; positively regulates anoikis [GO:0043276]